{
  "term_id": "GO:0072377",
  "term_label": "blood coagulation, common pathway",
  "gene_name": "Fibrinogen alpha chain",
  "gene": "UniProtKB:P02671",
  "gene_symbol": "FGA"
}